{
  "gene_symbol": "A0A0G2JKW9",
  "gene_name": "Uncharacterized protein",
  "term_id": "UNKNOWN:0003",
  "gene": "UniProtKB:A0A0G2JKW9",
  "term_label": "Unknown cellular component"
}